radial spoke head 1 [GO:0120336] (cellular component) Relationships: is a type of GO:0001535; is part of radial spoke 1 [GO:0120333] References: PMID:22754630, PMID:348711799 Sources: GOC:krc Definition: The portion of the radial spoke 1 that is orthogonal to the elongated stalk and which projects towards the central pair of microtubules within the ciliary axoneme. Also known as: radial spokehead 1